{
  "term_id": "UNKNOWN:0002",
  "gene": "UniProtKB:Q96MR7",
  "term_label": "Unknown biological process",
  "gene_symbol": "OBSCN-AS1",
  "gene_name": "Putative uncharacterized protein OBSCN-AS1"
}